{
  "term_label": "myofibril assembly",
  "gene_name": "Neuralized-like protein 2",
  "gene": "UniProtKB:Q9BR09",
  "gene_symbol": "NEURL2",
  "term_id": "GO:0030239"
}